diaminopimelate decarboxylase activity [GO:0008836] (molecular function) Also known as: DAP decarboxylase activity, DAP-decarboxylase activity, diaminopimelic acid decarboxylase activity, meso-2,6-diaminoheptanedioate carboxy-lyase (L-lysine-forming), meso-2,6-diaminoheptanedioate carboxy-lyase activity, meso-diaminopimelate decarboxylase activity Relationships: is a type of GO:0016831 Sources: EC:4.1.1.20, RHEA:15101 Definition: Catalysis of the reaction: meso-2,6-diaminopimelate + H+ = L-lysine + CO2.